{
  "term_id": "GO:0038023",
  "gene": "UniProtKB:Q86UN3",
  "term_label": "signaling receptor activity",
  "gene_symbol": "RTN4RL2",
  "gene_name": "Reticulon-4 receptor-like 2"
}